{
  "gene_name": "Fibroblast growth factor 22",
  "gene": "UniProtKB:Q9HCT0",
  "gene_symbol": "FGF22",
  "term_id": "GO:0043410",
  "term_label": "positive regulation of MAPK cascade"
}